emericellamide biosynthetic process [GO:1900557] (biological process) Relationships: is a type of lipid biosynthetic process [GO:0008610]; is a type of secondary metabolite biosynthetic process [GO:0044550]; is a type of depsipeptide biosynthetic process [GO:0050763]; is a type of GO:0072339; is a type of lactone biosynthetic process [GO:1901336] Regulation: regulated by regulation of emericellamide biosynthetic process [GO:1900658]; negatively regulated by GO:1900659; positively regulated by positive regulation of emericellamide biosynthetic process [GO:1900660] Subtypes: GO:1900617 Sources: GOC:TermGenie, GOC:di Definition: The chemical reactions and pathways resulting in the formation of emericellamide. Also known as: emericellamide anabolism, emericellamide biosynthesis, emericellamide formation, emericellamide synthesis